{
  "term_id": "GO:0005634",
  "term_label": "nucleus",
  "gene": "UniProtKB:Q99932",
  "gene_symbol": "SPAG8",
  "gene_name": "Sperm-associated antigen 8"
}